{
  "gene_symbol": "TOMM70",
  "term_id": "GO:0005741",
  "term_label": "mitochondrial outer membrane",
  "gene": "UniProtKB:O94826",
  "gene_name": "Mitochondrial import receptor subunit TOM70"
}